{
  "term_id": "GO:0005940",
  "gene": "UniProtKB:Q9P0V9",
  "gene_name": "Septin-10",
  "gene_symbol": "SEPTIN10",
  "term_label": "septin ring"
}